negative regulation of nucleocytoplasmic transport [GO:0046823] (biological process) Also known as: down regulation of nucleocytoplasmic transport, down-regulation of nucleocytoplasmic transport, downregulation of nucleocytoplasmic transport, inhibition of nucleocytoplasmic transport Sources: GOC:bf Relationships: is a type of negative regulation of intracellular transport [GO:0032387]; is a type of GO:0046822; negatively regulates nucleocytoplasmic transport [GO:0006913] Subtypes: negative regulation of protein import into nucleus [GO:0042308], negative regulation of protein export from nucleus [GO:0046826], negative regulation of RNA import into nucleus [GO:0046829], negative regulation of RNA export from nucleus [GO:0046832], negative regulation of ribosomal subunit export from nucleus [GO:2000201] Definition: Any process that stops, prevents, or reduces the frequency, rate or extent of the directed movement of substances between the cytoplasm and the nucleus.